vitamin A import into cell [GO:0071939] (biological process) Definition: The directed movement of vitamin A from outside of a cell, across the plasma membrane and into the cytosol. Vitamin A is any of several retinoid derivatives of beta-carotene, primarily retinol, retinal, or retinoic acid. References: PMID:16011460, PMID:1924551 Sources: GOC:mah Also known as: vitamin A uptake, vitamin A import Relationships: is_a vitamin transmembrane transport [GO:0035461]; is a type of vitamin A transport [GO:0071938]; is a type of import into cell [GO:0098657]; is a type of lipid import into cell [GO:0140354]